{
  "gene_symbol": "IRX6",
  "term_id": "GO:0030182",
  "term_label": "neuron differentiation",
  "gene_name": "Iroquois-class homeodomain protein IRX-6",
  "gene": "UniProtKB:P78412"
}